{
  "gene": "UniProtKB:Q9P0L0",
  "gene_symbol": "VAPA",
  "gene_name": "Vesicle-associated membrane protein-associated protein A",
  "term_id": "GO:0005886",
  "term_label": "plasma membrane"
}